{
  "term_id": "GO:0070411",
  "gene": "UniProtKB:Q15797",
  "gene_name": "Mothers against decapentaplegic homolog 1",
  "term_label": "I-SMAD binding",
  "gene_symbol": "SMAD1"
}